positive regulation of humoral immune response mediated by circulating immunoglobulin [GO:0002925] (biological process) Sources: GOC:add Also known as: up regulation of humoral immune response mediated by circulating immunoglobulin, up-regulation of humoral immune response mediated by circulating immunoglobulin, upregulation of humoral immune response mediated by circulating immunoglobulin, activation of humoral immune response mediated by circulating immunoglobulin, stimulation of humoral immune response mediated by circulating immunoglobulin Definition: Any process that activates or increases the frequency, rate, or extent of a humoral immune response mediated by circulating immunoglobulin. Subtypes: positive regulation of complement activation, classical pathway [GO:0045960] Relationships: is a type of GO:0002891; is a type of positive regulation of humoral immune response [GO:0002922]; is a type of regulation of humoral immune response mediated by circulating immunoglobulin [GO:0002923]; positively regulates GO:0002455